{
  "term_id": "GO:0045944",
  "gene": "UniProtKB:Q9H2A3",
  "gene_name": "Neurogenin-2",
  "term_label": "positive regulation of transcription by RNA polymerase II",
  "gene_symbol": "NEUROG2"
}